{
  "gene": "UniProtKB:Q99828",
  "gene_name": "Calcium and integrin-binding protein 1",
  "term_id": "GO:0071363",
  "gene_symbol": "CIB1",
  "term_label": "cellular response to growth factor stimulus"
}